{
  "gene": "UniProtKB:P08118",
  "gene_symbol": "MSMB",
  "term_id": "UNKNOWN:0002",
  "gene_name": "Beta-microseminoprotein",
  "term_label": "Unknown biological process"
}